{
  "gene": "UniProtKB:Q7Z6J0",
  "gene_symbol": "SH3RF1",
  "term_label": "negative regulation of apoptotic process",
  "gene_name": "E3 ubiquitin-protein ligase SH3RF1",
  "term_id": "GO:0043066"
}